{
  "gene": "UniProtKB:Q9HAT1",
  "term_label": "endoplasmic reticulum to Golgi vesicle-mediated transport",
  "gene_name": "Protein ERGIC-53-like",
  "term_id": "GO:0006888",
  "gene_symbol": "LMAN1L"
}